{
  "gene_name": "Transmembrane protein 165",
  "term_id": "GO:0032472",
  "term_label": "Golgi calcium ion transport",
  "gene": "UniProtKB:Q9HC07",
  "gene_symbol": "TMEM165"
}